{
  "gene_name": "U11_U12 small nuclear ribonucleoprotein 48 kDa protein",
  "term_id": "GO:0005829",
  "gene": "UniProtKB:Q6IEG0",
  "term_label": "cytosol",
  "gene_symbol": "SNRNP48"
}